AMPA glutamate receptor complex [GO:0032281] (cellular component) Definition: An assembly of four or five subunits which form a structure with an extracellular N-terminus and a large loop that together form the ligand binding domain. The C-terminus is intracellular. The ionotropic glutamate receptor complex itself acts as a ligand gated ion channel; on binding glutamate, charged ions pass through a channel in the center of the receptor complex. The AMPA receptors mediate fast synaptic transmission in the CNS and are composed of subunits GluR1-4, products from separate genes. These subunits have an extracellular N-terminus and an intracellular C-terminus. Also known as: AMPA-selective glutamate receptor complex, alpha-amino-3-hydroxy-5-methyl-4-isoxazolepropionic acid selective glutamate receptor complex, AMPA receptor Relationships: is a type of ionotropic glutamate receptor complex [GO:0008328] Sources: GOC:ef